{
  "gene_symbol": "CYP4A11",
  "gene": "UniProtKB:Q02928",
  "gene_name": "Cytochrome P450 4A11",
  "term_id": "GO:0043651",
  "term_label": "linoleic acid metabolic process"
}